{
  "gene_name": "Immunoglobulin heavy variable 1-46",
  "term_label": "Unknown cellular component",
  "gene_symbol": "IGHV1-46",
  "gene": "UniProtKB:P01743",
  "term_id": "UNKNOWN:0003"
}